{
  "term_label": "Golgi apparatus",
  "gene": "UniProtKB:Q96K37",
  "gene_name": "Solute carrier family 35 member E1",
  "gene_symbol": "SLC35E1",
  "term_id": "GO:0005794"
}